{
  "gene_symbol": "YWHAQ",
  "gene": "UniProtKB:P27348",
  "term_label": "cytoplasm",
  "gene_name": "14-3-3 protein theta",
  "term_id": "GO:0005737"
}